{
  "term_id": "GO:0032956",
  "gene": "UniProtKB:Q6ZMC9",
  "gene_name": "Sialic acid-binding Ig-like lectin 15",
  "term_label": "regulation of actin cytoskeleton organization",
  "gene_symbol": "SIGLEC15"
}